{
  "gene": "UniProtKB:P12645",
  "term_id": "GO:0007178",
  "gene_name": "Bone morphogenetic protein 3",
  "term_label": "cell surface receptor protein serine/threonine kinase signaling pathway",
  "gene_symbol": "BMP3"
}